{
  "term_id": "UNKNOWN:0002",
  "term_label": "Unknown biological process",
  "gene": "UniProtKB:Q9Y4B6",
  "gene_symbol": "DCAF1",
  "gene_name": "DDB1- and CUL4-associated factor 1"
}